{
  "term_id": "GO:0006357",
  "gene_symbol": "BARHL1",
  "gene": "UniProtKB:Q9BZE3",
  "term_label": "regulation of transcription by RNA polymerase II",
  "gene_name": "BarH-like 1 homeobox protein"
}